{
  "term_id": "GO:0000139",
  "term_label": "Golgi membrane",
  "gene": "UniProtKB:Q9Y2D2",
  "gene_symbol": "SLC35A3",
  "gene_name": "UDP-N-acetylglucosamine transporter"
}